{
  "term_id": "GO:0005634",
  "gene_symbol": "BIRC7",
  "gene_name": "Baculoviral IAP repeat-containing protein 7",
  "gene": "UniProtKB:Q96CA5",
  "term_label": "nucleus"
}